{
  "gene_symbol": "GLIS1",
  "gene": "UniProtKB:Q8NBF1",
  "term_label": "RNA polymerase II cis-regulatory region sequence-specific DNA binding",
  "gene_name": "Zinc finger protein GLIS1",
  "term_id": "GO:0000978"
}